{
  "gene": "UniProtKB:O43247",
  "term_label": "Unknown cellular component",
  "gene_name": "Testis-expressed protein 33",
  "gene_symbol": "TEX33",
  "term_id": "UNKNOWN:0003"
}